oxidoreductase activity, acting on CH or CH2 groups, with an iron-sulfur protein as acceptor [GO:0052592] (MF) Definition: Catalysis of an oxidation-reduction (redox) reaction in which a CH2 group acts as a hydrogen or electron donor and reduces an iron-sulfur protein. Subtypes: GO:0046429, 4-hydroxy-3-methylbut-2-enyl diphosphate reductase activity [GO:0051745], 7-hydroxymethyl chlorophyll a reductase activity [GO:0090415], GO:0141197 Also known as: oxidoreductase activity, acting on CH or CH2 groups, with an iron-sulphur protein as acceptor Relationships: is a type of oxidoreductase activity, acting on CH or CH2 groups [GO:0016725] Sources: GOC:ai